dendrite extension [GO:0097484] (biological process) Sources: GOC:BHF, GOC:rl Relationships: is a type of neuron projection extension [GO:1990138] Definition: Long distance growth of a single dendrite involved in cellular development. Regulation: regulated by regulation of dendrite extension [GO:1903859]; negatively regulated by negative regulation of dendrite extension [GO:1903860]; positively regulated by positive regulation of dendrite extension [GO:1903861]